{
  "gene": "UniProtKB:P07148",
  "term_id": "GO:0005504",
  "gene_symbol": "FABP1",
  "term_label": "fatty acid binding",
  "gene_name": "Fatty acid-binding protein, liver"
}